maintenance of polarity of follicular epithelium [GO:0042248] (biological process) Relationships: is a type of establishment or maintenance of polarity of follicular epithelium [GO:0016334] Sources: GOC:bf Definition: The maintenance of an established polarized follicular epithelial sheet.